{
  "term_label": "RNA binding",
  "gene": "UniProtKB:Q8IYB3",
  "gene_symbol": "SRRM1",
  "term_id": "GO:0003723",
  "gene_name": "Serine_arginine repetitive matrix protein 1"
}